synephrine dehydratase activity [GO:0050315] (molecular function) Also known as: 1-(4-hydroxyphenyl)-2-(methylamino)ethanol hydro-lyase (methylamine-forming) Definition: Catalysis of the reaction: synephrine = (4-hydroxyphenyl)acetaldehyde + methylammonium. Sources: EC:4.2.1.88, RHEA:32203 Relationships: is a type of hydro-lyase activity [GO:0016836]